{
  "gene": "UniProtKB:A0A1B0GVT2",
  "gene_name": "Small integral membrane protein 36",
  "term_id": "UNKNOWN:0001",
  "gene_symbol": "SMIM36",
  "term_label": "Unknown molecular function"
}